{
  "gene_symbol": "GPHN",
  "term_id": "GO:0007529",
  "gene_name": "Gephyrin",
  "term_label": "establishment of synaptic specificity at neuromuscular junction",
  "gene": "UniProtKB:Q9NQX3"
}